{
  "gene": "UniProtKB:P33076",
  "term_label": "positive regulation of MHC class II biosynthetic process",
  "term_id": "GO:0045348",
  "gene_symbol": "CIITA",
  "gene_name": "MHC class II transactivator"
}